{
  "term_id": "GO:0007165",
  "gene_name": "Mitogen-activated protein kinase kinase kinase 10",
  "gene_symbol": "MAP3K10",
  "term_label": "signal transduction",
  "gene": "UniProtKB:Q02779"
}